{
  "gene_symbol": "ZNF23",
  "term_label": "nucleus",
  "gene_name": "Zinc finger protein 23",
  "gene": "UniProtKB:P17027",
  "term_id": "GO:0005634"
}